endocardial cushion to mesenchymal transition involved in heart chamber septation [GO:0003200] (biological process) Definition: A transition where an endocardial cell loses apical/basolateral polarity, severs intercellular adhesive junctions, degrades basement membrane components and becomes a migratory mesenchymal cell that will contribute to the formation of the heart septum. Relationships: is a type of GO:0090500; is part of cardiac septum morphogenesis [GO:0060411] Sources: GOC:mtg_heart